{
  "gene": "UniProtKB:O14796",
  "term_label": "Unknown cellular component",
  "gene_name": "SH2 domain-containing protein 1B",
  "term_id": "UNKNOWN:0003",
  "gene_symbol": "SH2D1B"
}